response to interleukin-21 [GO:0098756] (biological process) Also known as: response to IL-21 Subtypes: GO:0098757 Relationships: is a type of GO:0034097 Definition: Any process that results in a change in state or activity of a cell or an organism (in terms of movement, secretion, enzyme production, gene expression, etc.) as a result of an interleukin-21 stimulus. Sources: GOC:BHF, GOC:mah